negative regulation of digestive system process [GO:0060457] (biological process) Subtypes: negative regulation of hindgut contraction [GO:0060451], GO:0060455, negative regulation of pancreatic juice secretion [GO:0090188], negative regulation of small intestinal transit [GO:0120059], negative regulation of gastric emptying [GO:0120061], GO:1904479, negative regulation of saliva secretion [GO:1905747], negative regulation of defecation [GO:2000293] Definition: Any process that decreases the frequency, rate or extent of a digestive system process, a physical, chemical, or biochemical process carried out by living organisms to break down ingested nutrients into components that may be easily absorbed and directed into metabolism. Sources: GOC:dph, GOC:tb Relationships: is a type of regulation of digestive system process [GO:0044058]; is a type of negative regulation of multicellular organismal process [GO:0051241]; negatively regulates GO:0022600